{
  "gene": "UniProtKB:P10082",
  "gene_name": "Peptide YY",
  "term_label": "neuropeptide Y receptor binding",
  "gene_symbol": "PYY",
  "term_id": "GO:0031841"
}